{
  "gene_name": "Zinc finger CCHC domain-containing protein 3",
  "gene": "UniProtKB:Q9NUD5",
  "term_id": "GO:0002218",
  "gene_symbol": "ZCCHC3",
  "term_label": "activation of innate immune response"
}